spore-bearing structure formation [GO:0097751] (biological process) Definition: The process of generating a spore-bearing structure. A spore-bearing structure is an anatomical structure that produces new spores. Relationships: is a type of developmental process [GO:0032502]; is part of GO:0075259 Sources: GOC:di Also known as: sporangium formation, sporophore formation